negative regulation of relaxation of smooth muscle [GO:1901081] (biological process) Relationships: is a type of negative regulation of relaxation of muscle [GO:1901078]; is a type of regulation of relaxation of smooth muscle [GO:1901080]; negatively regulates relaxation of smooth muscle [GO:0044557] Subtypes: negative regulation of uterine smooth muscle relaxation [GO:1900720] Definition: Any process that stops, prevents or reduces the frequency, rate or extent of relaxation of smooth muscle. Also known as: down regulation of relaxation of smooth muscle, down regulation of smooth muscle relaxation, down-regulation of relaxation of smooth muscle, down-regulation of smooth muscle relaxation, downregulation of relaxation of smooth muscle, downregulation of smooth muscle relaxation, inhibition of smooth muscle relaxation, negative regulation of smooth muscle relaxation, inhibition of relaxation of smooth muscle Sources: GOC:TermGenie